{
  "term_id": "UNKNOWN:0001",
  "gene_symbol": "A8MZ25",
  "gene": "UniProtKB:A8MZ25",
  "term_label": "Unknown molecular function",
  "gene_name": "Putative uncharacterized protein FLJ38767"
}